indole-3-acetonitrile nitrile hydratase activity [GO:0080109] (molecular function) References: PMID:11607511, PMID:12430025 Sources: MetaCyc:RXN-7567 Relationships: is_a nitrile hydratase activity [GO:0018822] Definition: Catalysis of the reaction: indole-3-acetonitrile + H2O = indole-3-acetamide.